{
  "term_id": "UNKNOWN:0002",
  "gene": "UniProtKB:Q06250",
  "gene_name": "Putative Wilms tumor upstream neighbor 1 gene protein",
  "term_label": "Unknown biological process",
  "gene_symbol": "WT1-AS"
}